{
  "gene_name": "ATPase inhibitor, mitochondrial",
  "gene": "UniProtKB:Q9UII2",
  "gene_symbol": "ATP5IF1",
  "term_label": "erythrocyte differentiation",
  "term_id": "GO:0030218"
}